{
  "gene": "UniProtKB:Q6NSJ2",
  "gene_name": "Pleckstrin homology-like domain family B member 3",
  "gene_symbol": "PHLDB3",
  "term_label": "Unknown biological process",
  "term_id": "UNKNOWN:0002"
}